melanocyte apoptotic process [GO:1902362] (biological process) Also known as: melanocyte apoptosis, melanophore apoptosis, melanophore apoptotic process Relationships: is a type of GO:0006915 Definition: Any apoptotic process in a melanocyte, the main structural component of the epidermis. References: PMID:20530876 Sources: GOC:TermGenie, GOC:ic